{
  "gene": "UniProtKB:P49757",
  "term_id": "GO:0050769",
  "gene_name": "Protein numb homolog",
  "term_label": "positive regulation of neurogenesis",
  "gene_symbol": "NUMB"
}